U11 snRNA binding [GO:0030625] (molecular function) Definition: Binding to a U11 small nuclear RNA (U11 snRNA). Relationships: is a type of snRNA binding [GO:0017069] Sources: GOC:jl